{
  "gene": "UniProtKB:Q8TBG4",
  "gene_symbol": "ETNPPL",
  "term_id": "UNKNOWN:0003",
  "gene_name": "Ethanolamine-phosphate phospho-lyase",
  "term_label": "Unknown cellular component"
}